{
  "gene_name": "PHD finger-like domain-containing protein 5A",
  "term_id": "GO:0000398",
  "term_label": "mRNA splicing, via spliceosome",
  "gene": "UniProtKB:Q7RTV0",
  "gene_symbol": "PHF5A"
}